{
  "gene_symbol": "CCT8L1P",
  "gene_name": "Putative T-complex protein 1 subunit theta-like 1",
  "term_id": "GO:0005832",
  "gene": "UniProtKB:A6NM43",
  "term_label": "chaperonin-containing T-complex"
}